cytotoxic T cell differentiation [GO:0045065] (biological process) Sources: GOC:ai Note: Note that immunologists typically use the word 'development' to refer to cells of B or T cell lineages undergoing the process that GO describes as 'cell differentiation'. Regulation: RO_0002211 by regulation of cytotoxic T cell differentiation [GO:0045583]; negatively regulated by negative regulation of cytotoxic T cell differentiation [GO:0045584]; positively regulated by positive regulation of cytotoxic T cell differentiation [GO:0045585] Definition: The process in which a relatively unspecialized T cell acquires specialized features of a cytotoxic T cell. Also known as: cytotoxic T lymphocyte selection, cytotoxic T-cell selection, cytotoxic T-lymphocyte selection, cytotoxic T cell development Relationships: is a type of GO:0030217 Subtypes: CD8-positive, alpha-beta cytotoxic T cell differentiation [GO:0002308]